{
  "gene_symbol": "PIH1D1",
  "term_label": "R2TP complex",
  "gene": "UniProtKB:Q9NWS0",
  "term_id": "GO:0097255",
  "gene_name": "PIH1 domain-containing protein 1"
}